{
  "gene": "UniProtKB:Q9NZ81",
  "gene_symbol": "PRR13",
  "term_id": "GO:0005654",
  "term_label": "nucleoplasm",
  "gene_name": "Proline-rich protein 13"
}